negative regulation of AMPA glutamate receptor clustering [GO:1904718] (biological process) References: PMID:21558424 Sources: GOC:TermGenie, GOC:hjd, GO_REF:0000058 Also known as: down regulation of AMPA glutamate receptor clustering, down regulation of AMPA receptor clustering, down regulation of alpha-amino-3-hydroxy-5-methyl-4-isoxazole propionate selective glutamate receptor clustering, down-regulation of AMPA glutamate receptor clustering, down-regulation of AMPA receptor clustering, down-regulation of alpha-amino-3-hydroxy-5-methyl-4-isoxazole propionate selective glutamate receptor clustering, downregulation of AMPA glutamate receptor clustering, downregulation of AMPA receptor clustering, downregulation of alpha-amino-3-hydroxy-5-methyl-4-isoxazole propionate selective glutamate receptor clustering, negative regulation of AMPA receptor clustering, negative regulation of alpha-amino-3-hydroxy-5-methyl-4-isoxazole propionate selective glutamate receptor clustering, inhibition of AMPA glutamate receptor clustering, inhibition of AMPA receptor clustering, inhibition of alpha-amino-3-hydroxy-5-methyl-4-isoxazole propionate selective glutamate receptor clustering Relationships: is a type of negative regulation of postsynaptic membrane organization [GO:1901627]; is a type of GO:1903910; is a type of regulation of AMPA glutamate receptor clustering [GO:1904717]; negatively regulates AMPA glutamate receptor clustering [GO:0097113] Definition: Any process that stops, prevents or reduces the frequency, rate or extent of AMPA glutamate receptor clustering.